negative regulation of compound eye cone cell fate specification [GO:0042683] (biological process) Relationships: is a type of negative regulation of cell fate specification [GO:0009996]; is a type of regulation of compound eye cone cell fate specification [GO:0042682]; negatively regulates compound eye cone cell fate specification [GO:0042679] Sources: GOC:mtg_sensu Also known as: down regulation of cone cell fate specification, down-regulation of cone cell fate specification, downregulation of cone cell fate specification, inhibition of cone cell fate specification, suppression of cone cell fate Definition: Any process that restricts, stops or prevents a cell from specifying into a compound eye cone cell.